{
  "gene": "UniProtKB:Q8WZA2",
  "gene_symbol": "RAPGEF4",
  "gene_name": "Rap guanine nucleotide exchange factor 4",
  "term_id": "GO:0005886",
  "term_label": "plasma membrane"
}